{
  "gene_symbol": "PROSER2",
  "term_id": "UNKNOWN:0002",
  "gene": "UniProtKB:Q86WR7",
  "gene_name": "Proline and serine-rich protein 2",
  "term_label": "Unknown biological process"
}